{
  "term_label": "mRNA splicing, via spliceosome",
  "gene_name": "RNA-binding motif protein, X-linked-like-3",
  "term_id": "GO:0000398",
  "gene": "UniProtKB:Q8N7X1",
  "gene_symbol": "RBMXL3"
}